{
  "gene": "UniProtKB:Q8N6R0",
  "term_label": "Unknown cellular component",
  "gene_symbol": "METTL13",
  "gene_name": "eEF1A lysine and N-terminal methyltransferase",
  "term_id": "UNKNOWN:0003"
}